{
  "gene": "UniProtKB:Q8TEQ8",
  "gene_symbol": "PIGO",
  "term_id": "GO:0005789",
  "term_label": "endoplasmic reticulum membrane",
  "gene_name": "GPI ethanolamine phosphate transferase 3"
}